trans-synaptic signaling by nitric oxide [GO:0099548] (biological process) Sources: GOC:dos Definition: Cell-cell signaling between presynapse and postsynapse mediated by nitric oxide. Relationships: is_a synaptic signaling by nitric oxide [GO:0099163]; is a type of GO:0099543 Subtypes: retrograde trans-synaptic signaling by nitric oxide [GO:0098924], anterograde trans-synaptic signaling by nitric oxide [GO:0098940], trans-synaptic signaling by nitric oxide, modulating synaptic transmission [GO:0099555]